{
  "gene": "UniProtKB:A5X5Y0",
  "term_id": "GO:1904315",
  "term_label": "transmitter-gated monoatomic ion channel activity involved in regulation of postsynaptic membrane potential",
  "gene_name": "5-hydroxytryptamine receptor 3E",
  "gene_symbol": "HTR3E"
}